{
  "gene": "UniProtKB:Q9Y5Y9",
  "gene_name": "Sodium channel protein type 10 subunit alpha",
  "term_id": "GO:0001518",
  "term_label": "voltage-gated sodium channel complex",
  "gene_symbol": "SCN10A"
}